{
  "gene": "UniProtKB:P11684",
  "term_id": "UNKNOWN:0001",
  "gene_symbol": "SCGB1A1",
  "term_label": "Unknown molecular function",
  "gene_name": "Uteroglobin"
}